alpha4-beta1 integrin-paxillin complex [GO:0071102] (cellular component) Also known as: ITGA4-ITGB1-PXN complex Definition: A protein complex that consists of an alpha4-beta1 integrin complex bound to paxillin. References: PMID:12221126 Relationships: is a type of plasma membrane protein complex [GO:0098797]